dTTP metabolic process [GO:0046075] (biological process) Relationships: is a type of pyrimidine deoxyribonucleoside triphosphate metabolic process [GO:0009211]; is a type of pyrimidine deoxyribonucleotide metabolic process [GO:0009219] Definition: The chemical reactions and pathways involving dTTP, deoxyribosylthymine triphosphate. Also known as: dTTP metabolism Sources: GOC:go_curators Subtypes: GO:0006235, GO:0046076